{
  "gene_symbol": "FNDC10",
  "term_label": "Unknown biological process",
  "term_id": "UNKNOWN:0002",
  "gene": "UniProtKB:F2Z333",
  "gene_name": "Fibronectin type III domain-containing protein 10"
}